{
  "gene_symbol": "TUBAL3",
  "term_id": "GO:0005525",
  "gene": "UniProtKB:A6NHL2",
  "gene_name": "Tubulin alpha chain-like 3",
  "term_label": "GTP binding"
}